{
  "gene_name": "Zinc finger protein 302",
  "gene": "UniProtKB:Q9NR11",
  "gene_symbol": "ZNF302",
  "term_id": "GO:0005634",
  "term_label": "nucleus"
}